{
  "term_label": "nucleus",
  "gene": "UniProtKB:Q96L96",
  "term_id": "GO:0005634",
  "gene_symbol": "ALPK3",
  "gene_name": "Alpha-protein kinase 3"
}